{
  "term_label": "endoplasmic reticulum",
  "gene": "UniProtKB:Q8IVQ6",
  "term_id": "GO:0005783",
  "gene_symbol": "ZDHHC21",
  "gene_name": "Palmitoyltransferase ZDHHC21"
}